{
  "term_id": "GO:0008431",
  "term_label": "vitamin E binding",
  "gene_name": "Alpha-tocopherol transfer protein",
  "gene": "UniProtKB:P49638",
  "gene_symbol": "TTPA"
}